phenol-containing compound catabolic process [GO:0019336] (biological process) Definition: The chemical reactions and pathways resulting in the breakdown of a phenol, any compound containing one or more hydroxyl groups directly attached to an aromatic carbon ring. Sources: ISBN:0198506732 Also known as: phenol-containing compound breakdown, phenol-containing compound catabolism, phenol-containing compound degradation Subtypes: pentachlorophenol catabolic process [GO:0019338], gallate catabolic process [GO:0019396], GO:0019599, 3-hydroxyphenylacetate catabolic process [GO:0019610], catechol-containing compound catabolic process [GO:0019614], curcumin catabolic process [GO:0036040], asperthecin catabolic process [GO:0036183], vanillin catabolic process [GO:0042190], GO:0042209, GO:0042404, serotonin catabolic process [GO:0042429], eugenol catabolic process [GO:0042856], GO:0042865, bisphenol A catabolic process [GO:0043636], melanin catabolic process [GO:0046150], aerobic phenol-containing compound catabolic process [GO:0046191], anaerobic phenol-containing compound catabolic process [GO:0046193], 4-nitrophenol catabolic process [GO:0046196], cresol catabolic process [GO:0046199], GO:0046244, octopamine catabolic process [GO:0046334], diorcinol catabolic process [GO:1900571], emodin catabolic process [GO:1900574], o-orsellinic acid catabolic process [GO:1900583], endocrocin catabolic process [GO:1900601], F-9775A catabolic process [GO:1900610], GO:1900613, averantin catabolic process [GO:1900762], emericellin catabolic process [GO:1900765], fonsecin catabolic process [GO:1900768], shamixanthone catabolic process [GO:1900792], GO:1900814, 4-hydroxyphenylacetate catabolic process [GO:1901023], ferulate catabolic process [GO:1901067], funalenone catabolic process [GO:1901365], GO:1901886, homogentisate catabolic process [GO:1902000], neosartoricin catabolic process [GO:1902049], (-)-pinoresinol catabolic process [GO:1902123], GO:1902125, GO:1902128, GO:1902131, GO:1902134, GO:1902137 Relationships: is a type of catabolic process [GO:0009056]; is a type of phenol-containing compound metabolic process [GO:0018958]